{
  "term_label": "nucleus",
  "gene_symbol": "EIF2AK1",
  "gene": "UniProtKB:Q9BQI3",
  "gene_name": "Eukaryotic translation initiation factor 2-alpha kinase 1",
  "term_id": "GO:0005634"
}